{
  "gene": "UniProtKB:Q6ZS62",
  "gene_symbol": "COLCA1",
  "term_id": "UNKNOWN:0002",
  "gene_name": "Colorectal cancer-associated protein 1",
  "term_label": "Unknown biological process"
}